{
  "term_id": "GO:0015630",
  "gene": "UniProtKB:Q8NDL9",
  "gene_name": "Cytosolic carboxypeptidase-like protein 5",
  "gene_symbol": "AGBL5",
  "term_label": "microtubule cytoskeleton"
}